{
  "gene_name": "Insulin-induced gene 2 protein",
  "term_label": "cholesterol biosynthetic process",
  "term_id": "GO:0006695",
  "gene_symbol": "INSIG2",
  "gene": "UniProtKB:Q9Y5U4"
}